{
  "term_label": "cytokine activity",
  "gene_name": "Oncostatin-M",
  "gene": "UniProtKB:P13725",
  "term_id": "GO:0005125",
  "gene_symbol": "OSM"
}